{
  "gene_name": "cTAGE family member 2",
  "term_label": "endoplasmic reticulum exit site",
  "gene": "UniProtKB:Q96RT6",
  "term_id": "GO:0070971",
  "gene_symbol": "CTAGE1"
}